{
  "gene_name": "Solute carrier organic anion transporter family member 4A1",
  "term_label": "sodium-independent organic anion transport",
  "gene_symbol": "SLCO4A1",
  "term_id": "GO:0043252",
  "gene": "UniProtKB:Q96BD0"
}